{
  "term_label": "Unknown biological process",
  "gene_symbol": "PRAC1",
  "term_id": "UNKNOWN:0002",
  "gene_name": "Small nuclear protein PRAC1",
  "gene": "UniProtKB:Q96KF2"
}